{
  "gene_name": "Beta-soluble NSF attachment protein",
  "term_label": "regulation of synaptic vesicle priming",
  "term_id": "GO:0010807",
  "gene_symbol": "NAPB",
  "gene": "UniProtKB:Q9H115"
}